{
  "term_id": "UNKNOWN:0002",
  "gene_symbol": "NAA38",
  "term_label": "Unknown biological process",
  "gene_name": "N-alpha-acetyltransferase 38, NatC auxiliary subunit",
  "gene": "UniProtKB:Q9BRA0"
}